{
  "term_label": "spindle midzone",
  "gene_symbol": "RACGAP1",
  "gene_name": "Rac GTPase-activating protein 1",
  "gene": "UniProtKB:Q9H0H5",
  "term_id": "GO:0051233"
}